{
  "gene": "UniProtKB:Q12972",
  "term_id": "GO:0016607",
  "term_label": "nuclear speck",
  "gene_symbol": "PPP1R8",
  "gene_name": "Nuclear inhibitor of protein phosphatase 1"
}